{
  "term_label": "Unknown molecular function",
  "term_id": "UNKNOWN:0001",
  "gene_symbol": "EFCAB7",
  "gene_name": "EF-hand calcium-binding domain-containing protein 7",
  "gene": "UniProtKB:A8K855"
}